{
  "term_id": "UNKNOWN:0001",
  "term_label": "Unknown molecular function",
  "gene": "UniProtKB:Q9NNZ3",
  "gene_name": "DnaJ homolog subfamily C member 4",
  "gene_symbol": "DNAJC4"
}